{
  "gene_name": "Growth_differentiation factor 7",
  "term_label": "extracellular space",
  "gene": "UniProtKB:Q7Z4P5",
  "term_id": "GO:0005615",
  "gene_symbol": "GDF7"
}